cortical endoplasmic reticulum [GO:0032541] (cellular component) Relationships: is a type of endoplasmic reticulum tubular network [GO:0071782]; is part of cell cortex [GO:0005938] Also known as: ER-PM peripheral junction, cortical ER, peripheral ER, peripheral endoplasmic reticulum Definition: A cortical network of highly dynamic tubules that are juxtaposed to the plasma membrane and undergo ring closure and tubule-branching movements. Note: The dynamic nature of the cortical ER and the movements it undergoes (branching and ring closure) has been shown in both yeast and mammalian cells, so appears highly conserved. (PMID:10931860) References: PMID:10931860, PMID:17686782 Sources: GOC:se